{
  "gene_symbol": "CTPS1",
  "term_label": "identical protein binding",
  "gene": "UniProtKB:P17812",
  "gene_name": "CTP synthase 1",
  "term_id": "GO:0042802"
}